{
  "term_label": "Unknown biological process",
  "gene": "UniProtKB:A6QL63",
  "term_id": "UNKNOWN:0002",
  "gene_name": "Ankyrin repeat and BTB_POZ domain-containing protein 3",
  "gene_symbol": "ABTB3"
}